{
  "gene": "UniProtKB:O94964",
  "term_id": "GO:0008286",
  "term_label": "insulin receptor signaling pathway",
  "gene_name": "Protein SOGA1",
  "gene_symbol": "SOGA1"
}